{
  "term_id": "UNKNOWN:0002",
  "gene_symbol": "SMRP1",
  "term_label": "Unknown biological process",
  "gene_name": "Spermatid-specific manchette-related protein 1",
  "gene": "UniProtKB:Q8NCR6"
}